mesenchymal stem cell maintenance involved in mesonephric nephron morphogenesis [GO:0061235] (biological process) Relationships: is a type of GO:0072038; is part of mesonephric nephron morphogenesis [GO:0061228] Regulation: regulated by regulation of mesenchymal cell apoptotic process involved in mesonephric nephron morphogenesis [GO:0061295]; negatively regulated by negative regulation of mesenchymal cell apoptotic process involved in mesonephric nephron morphogenesis [GO:0061296]; positively regulated by positive regulation of mesenchymal cell apoptotic process involved in mesonephric nephron morphogenesis [GO:0061297] Sources: GOC:mtg_kidney_jan10 Definition: The process in which an organism retains a population of mesenchymal stem cells that contributes to the shaping of a nephron in the mesonephros. A mesenchymal stem cell is a cell that retains the ability to divide and proliferate throughout life to provide progenitor cells that can differentiate into specialized mesenchymal cells.